{
  "term_id": "GO:0141069",
  "gene_symbol": "TMEFF1",
  "gene_name": "Tomoregulin-1",
  "term_label": "receptor ligand inhibitor activity",
  "gene": "UniProtKB:Q8IYR6"
}